{
  "term_id": "UNKNOWN:0001",
  "term_label": "Unknown molecular function",
  "gene": "UniProtKB:Q92572",
  "gene_symbol": "AP3S1",
  "gene_name": "AP-3 complex subunit sigma-1"
}